{
  "gene_name": "Double homeobox protein A",
  "gene": "UniProtKB:A6NLW8",
  "term_id": "GO:0005634",
  "term_label": "nucleus",
  "gene_symbol": "DUXA"
}